{
  "gene_symbol": "EPB41",
  "term_id": "GO:0005856",
  "gene": "UniProtKB:P11171",
  "term_label": "cytoskeleton",
  "gene_name": "Protein 4.1"
}